{
  "term_label": "adherens junction",
  "gene": "UniProtKB:P55291",
  "gene_name": "Cadherin-15",
  "gene_symbol": "CDH15",
  "term_id": "GO:0005912"
}